{
  "term_label": "signal transduction",
  "term_id": "GO:0007165",
  "gene_name": "Contactin-associated protein 1",
  "gene_symbol": "CNTNAP1",
  "gene": "UniProtKB:P78357"
}